negative regulation of branchiomeric skeletal muscle development [GO:0014713] (biological process) Sources: GOC:mtg_muscle Relationships: is a type of regulation of branchiomeric skeletal muscle development [GO:0014711]; is a type of GO:0048642; negatively regulates branchiomeric skeletal muscle development [GO:0014707] Definition: Any process that stops, prevents, or reduces the frequency, rate or extent of branchiomeric skeletal muscle development. Branchiomeric skeletal muscle development is the process whose specific outcome is the progression of the branchiomeric skeletal muscle over time, from its formation to the mature structure.